{
  "gene_name": "Iron-sulfur protein NUBPL",
  "term_id": "GO:0005739",
  "gene_symbol": "NUBPL",
  "gene": "UniProtKB:Q8TB37",
  "term_label": "mitochondrion"
}